alkyne catabolic process [GO:0043454] (biological process) Also known as: alkyne breakdown, alkyne catabolism, alkyne degradation Definition: The chemical reactions and pathways resulting in the breakdown of an alkyne, any acyclic branched or unbranched hydrocarbon (compound composed only of carbon and hydrogen) having a carbon-carbon triple bond and the general formula CnH2n-2. Subtypes: GO:0019487 Sources: GOC:jl, GOC:krc, Wikipedia:Alkyne Relationships: is a type of hydrocarbon catabolic process [GO:0120253]